{
  "gene": "UniProtKB:Q9BZF9",
  "term_id": "GO:0008631",
  "term_label": "intrinsic apoptotic signaling pathway in response to oxidative stress",
  "gene_name": "Uveal autoantigen with coiled-coil domains and ankyrin repeats",
  "gene_symbol": "UACA"
}